{
  "term_id": "GO:0005739",
  "term_label": "mitochondrion",
  "gene": "UniProtKB:P25325",
  "gene_name": "3-mercaptopyruvate sulfurtransferase",
  "gene_symbol": "MPST"
}